embryonic cardiac muscle cell growth involved in heart morphogenesis [GO:0003246] (biological process) Definition: The growth of a cardiac muscle cell during the embryonic period, that contributes to the shaping of the heart. Relationships: is a type of growth involved in heart morphogenesis [GO:0003241]; is a type of GO:0061049; is part of cardiac muscle tissue growth involved in heart morphogenesis [GO:0003245] Sources: GOC:mtg_heart Also known as: embryonic cardiac muscle physiological hypertrophy